{
  "term_id": "GO:0061617",
  "term_label": "MICOS complex",
  "gene_name": "MICOS complex subunit MIC13",
  "gene_symbol": "MICOS13",
  "gene": "UniProtKB:Q5XKP0"
}